{
  "gene_name": "Misshapen-like kinase 1",
  "term_id": "GO:0048812",
  "gene": "UniProtKB:Q8N4C8",
  "gene_symbol": "MINK1",
  "term_label": "neuron projection morphogenesis"
}